{
  "gene_symbol": "LAMB4",
  "gene": "UniProtKB:A4D0S4",
  "gene_name": "Laminin subunit beta-4",
  "term_label": "substrate adhesion-dependent cell spreading",
  "term_id": "GO:0034446"
}